{
  "term_id": "UNKNOWN:0001",
  "gene_symbol": "TCP11L1",
  "term_label": "Unknown molecular function",
  "gene": "UniProtKB:Q9NUJ3",
  "gene_name": "T-complex protein 11-like protein 1"
}